{
  "gene": "UniProtKB:Q8N9F7",
  "term_id": "GO:0008081",
  "gene_symbol": "GDPD1",
  "term_label": "phosphoric diester hydrolase activity",
  "gene_name": "Lysophospholipase D GDPD1"
}